olfactory nerve formation [GO:0021628] (biological process) Relationships: is a type of cranial nerve formation [GO:0021603]; is part of GO:0021627 Also known as: CN I biosynthesis, CN I formation Sources: GOC:cls, GOC:dgh, GOC:dph, GOC:jid, GO_REF:0000021 Definition: The process that gives rise to the olfactory nerve. This process pertains to the initial formation of a structure from unspecified parts. The olfactory nerve is a collection of sensory nerve rootlets that extend down from the olfactory bulb to the olfactory mucosa of the upper parts of the nasal cavity. This nerve conducts odor information to the brainstem.